hindbrain-spinal cord boundary formation [GO:0021906] (biological process) Definition: The process whose specific outcome is the formation of the hindbrain-spinal cord boundary. References: PMID:11262869 Sources: GOC:cls, GOC:dgh, GOC:dph, GOC:jid, GO_REF:0000021 Relationships: is a type of formation of anatomical boundary [GO:0048859]; is part of rostrocaudal neural tube patterning [GO:0021903]